{
  "term_id": "GO:0034185",
  "gene_name": "Lipoprotein lipase",
  "gene": "UniProtKB:P06858",
  "gene_symbol": "LPL",
  "term_label": "apolipoprotein binding"
}